{
  "gene": "UniProtKB:Q96IR2",
  "gene_name": "Zinc finger protein 845",
  "gene_symbol": "ZNF845",
  "term_id": "GO:0000122",
  "term_label": "negative regulation of transcription by RNA polymerase II"
}